negative regulation of starch utilization system complex assembly [GO:1900513] (biological process) Relationships: is a type of negative regulation of protein-containing complex assembly [GO:0031333]; is a type of regulation of starch utilization system complex assembly [GO:1900512]; negatively regulates GO:0044574 Sources: GOC:TermGenie, GOC:mengo_curators Definition: Any process that stops, prevents or reduces the frequency, rate or extent of starch utilization system complex assembly. Also known as: down regulation of SUS complex assembly, down regulation of assembly of starch utilization system complex, down regulation of starch utilization system complex assembly, down-regulation of SUS complex assembly, down-regulation of assembly of starch utilization system complex, down-regulation of starch utilization system complex assembly, downregulation of SUS complex assembly, downregulation of assembly of starch utilization system complex, downregulation of starch utilization system complex assembly, inhibition of SUS complex assembly, inhibition of assembly of starch utilization system complex, negative regulation of SUS complex assembly, negative regulation of assembly of starch utilization system complex, inhibition of starch utilization system complex assembly